pyridoxine transmembrane transport [GO:1903092] (BP) References: PMID:15701794 Sources: GOC:TermGenie, GO_REF:0000069 Relationships: is a type of pyridoxine transport [GO:0031923]; is a type of vitamin transmembrane transport [GO:0035461] Definition: The process in which pyridoxine is transported across a membrane. Subtypes: pyridoxine import across plasma membrane [GO:1903075]